{
  "term_id": "GO:0006369",
  "gene": "UniProtKB:P24928",
  "term_label": "termination of RNA polymerase II transcription",
  "gene_symbol": "POLR2A",
  "gene_name": "DNA-directed RNA polymerase II subunit RPB1"
}